cinnamoyl-CoA:phenyllactate CoA-transferase activity [GO:0043785] (molecular function) Also known as: (E)-cinnamoyl-CoA:(R)-phenyllactate CoA-transferase activity, FldA Definition: Catalysis of the reaction: (R)-3-phenyllactate + [(2R,3S,4R,5R)-5-(6-amino-9H-purin-9-yl)-4-hydroxy-3-(phosphonatooxy)oxolan-2-yl]methyl {[(3R)-3-hydroxy-2,2-dimethyl-3-({2-[(2-{[(2E)-3-phenylprop-2-enoyl]sulfanyl}ethyl)carbamoyl]ethyl}carbamoyl)propyl phosphonato]oxy}phosphonate = (R)-3-phenyllactoyl-CoA + trans-cinnamate. Sources: EC:2.8.3.17, RHEA:15601 Relationships: is a type of GO:0008410